{
  "gene_symbol": "ECHDC1",
  "term_label": "fatty acid beta-oxidation",
  "gene": "UniProtKB:Q9NTX5",
  "gene_name": "Ethylmalonyl-CoA decarboxylase",
  "term_id": "GO:0006635"
}